NADPH-cytochrome-c2 reductase activity [GO:0015047] (molecular function) Sources: EC:1.6.2.5 Relationships: is a type of oxidoreductase activity, acting on NAD(P)H, heme protein as acceptor [GO:0016653] Definition: Catalysis of the reaction: NADPH + H+ + 2 ferricytochrome c2 = NADP+ + 2 ferrocytochrome c2. Also known as: NADPH:ferricytochrome-c2 oxidoreductase activity, cytochrome c2 reductase (reduced nicotinamide adinine dinucleotide phosphate, NADPH), reductase, cytochrome c2 (reduced nicotinamide adenine dinucleotide phosphate)